{
  "term_id": "UNKNOWN:0001",
  "gene_name": "Cytokine-like protein 1",
  "gene_symbol": "CYTL1",
  "term_label": "Unknown molecular function",
  "gene": "UniProtKB:Q9NRR1"
}